acetyltransferase complex [GO:1902493] (CC) Relationships: is a type of transferase complex [GO:1990234] References: PMID:8077207 Sources: GOC:TermGenie, GOC:bhm Definition: A protein complex which is capable of acetyltransferase activity. Subtypes: protein acetyltransferase complex [GO:0031248], GO:0045254, diamine N-acetyltransferase complex [GO:1990235]